{
  "term_label": "exocyst",
  "term_id": "GO:0000145",
  "gene_name": "Exocyst complex component 4",
  "gene_symbol": "EXOC4",
  "gene": "UniProtKB:Q96A65"
}